{
  "term_id": "GO:0050955",
  "gene_name": "Transient receptor potential cation channel subfamily A member 1",
  "term_label": "thermoception",
  "gene_symbol": "TRPA1",
  "gene": "UniProtKB:O75762"
}